{
  "gene_name": "T cell receptor alpha variable 8-7 (pseudogene) (Fragment)",
  "term_label": "immunoglobulin complex",
  "term_id": "GO:0019814",
  "gene": "UniProtKB:A0A075B6U6",
  "gene_symbol": "TRAV8-7"
}